{
  "term_id": "GO:0004563",
  "term_label": "beta-N-acetylhexosaminidase activity",
  "gene": "UniProtKB:P07686",
  "gene_name": "Beta-hexosaminidase subunit beta",
  "gene_symbol": "HEXB"
}